{
  "gene": "UniProtKB:Q8IUA0",
  "term_id": "UNKNOWN:0001",
  "gene_name": "WAP four-disulfide core domain protein 8",
  "gene_symbol": "WFDC8",
  "term_label": "Unknown molecular function"
}